{
  "gene": "UniProtKB:Q92832",
  "gene_name": "Protein kinase C-binding protein NELL1",
  "gene_symbol": "NELL1",
  "term_label": "heparin binding",
  "term_id": "GO:0008201"
}